{
  "gene_name": "Serine_threonine-protein kinase WNK1",
  "term_label": "intracellular signal transduction",
  "gene": "UniProtKB:Q9H4A3",
  "gene_symbol": "WNK1",
  "term_id": "GO:0035556"
}